{
  "gene_name": "[F-actin]-monooxygenase MICAL1",
  "gene_symbol": "MICAL1",
  "gene": "UniProtKB:Q8TDZ2",
  "term_label": "actin cytoskeleton",
  "term_id": "GO:0015629"
}